{
  "gene": "UniProtKB:Q8TCZ2",
  "term_id": "UNKNOWN:0003",
  "term_label": "Unknown cellular component",
  "gene_symbol": "CD99L2",
  "gene_name": "CD99 antigen-like protein 2"
}